{
  "term_label": "MAP kinase phosphatase activity",
  "gene_symbol": "DUSP26",
  "gene": "UniProtKB:Q9BV47",
  "gene_name": "Dual specificity protein phosphatase 26",
  "term_id": "GO:0033549"
}